{
  "term_id": "GO:0003779",
  "term_label": "actin binding",
  "gene": "UniProtKB:P15311",
  "gene_symbol": "EZR",
  "gene_name": "Ezrin"
}